positive regulation of stress granule assembly [GO:0062029] (biological process) Definition: Any process that starts or increases the rate, frequency or extent of stress-granule assembly, the aggregation, arrangement and bonding together of proteins and RNA molecules to form a stress granule. References: PMID:20180778 Relationships: is a type of regulation of stress granule assembly [GO:0062028]; is a type of positive regulation of organelle assembly [GO:1902117]; positively regulates stress granule assembly [GO:0034063]